{
  "gene_name": "SERTA domain-containing protein 4",
  "gene_symbol": "SERTAD4",
  "gene": "UniProtKB:Q9NUC0",
  "term_label": "Unknown molecular function",
  "term_id": "UNKNOWN:0001"
}